{
  "term_id": "GO:0030317",
  "term_label": "flagellated sperm motility",
  "gene_symbol": "DNAAF6",
  "gene_name": "Dynein axonemal assembly factor 6",
  "gene": "UniProtKB:Q9NQM4"
}